positive regulation of triglyceride catabolic process [GO:0010898] (biological process) Definition: Any process that increases the frequency, rate, or extent of the chemical reactions and pathways resulting in the breakdown of triglyceride. Sources: GOC:rn, GOC:tb Relationships: is a type of regulation of triglyceride catabolic process [GO:0010896]; is a type of positive regulation of lipid catabolic process [GO:0050996]; is a type of positive regulation of triglyceride metabolic process [GO:0090208]; positively regulates triglyceride catabolic process [GO:0019433] Also known as: positive regulation of triacylglycerol catabolic process